{
  "term_label": "protein polyubiquitination",
  "gene_symbol": "UBE2J1",
  "gene": "UniProtKB:Q9Y385",
  "gene_name": "Ubiquitin-conjugating enzyme E2 J1",
  "term_id": "GO:0000209"
}